{
  "gene": "UniProtKB:Q6IF82",
  "gene_symbol": "OR4A47",
  "term_label": "Unknown biological process",
  "gene_name": "Olfactory receptor 4A47",
  "term_id": "UNKNOWN:0002"
}